{
  "term_label": "plasma membrane",
  "gene_symbol": "RHO",
  "term_id": "GO:0005886",
  "gene_name": "Rhodopsin",
  "gene": "UniProtKB:P08100"
}